clathrin-sculpted acetylcholine transport vesicle lumen [GO:0060202] (cellular component) Also known as: clathrin sculpted acetylcholine constitutive secretory pathway transport vesicle lumen, clathrin sculpted acetylcholine transport vesicle lumen Sources: GOC:dph Definition: The volume enclosed by the membrane of the clathrin-sculpted acetylcholine transport vesicle. Relationships: is a type of cytoplasmic vesicle lumen [GO:0060205]; is part of clathrin-sculpted acetylcholine transport vesicle [GO:0060200]